{
  "gene_name": "Contactin-4",
  "gene": "UniProtKB:Q8IWV2",
  "term_label": "homophilic cell-cell adhesion",
  "gene_symbol": "CNTN4",
  "term_id": "GO:0007156"
}